heparan sulfate N-sulfotransferase activity [GO:0015016] (molecular function) Definition: Catalysis of the reaction: 3'-phosphoadenylyl sulfate + alpha-D-glucosaminyl-[heparan sulfate](n) = adenosine 3',5'-bisphosphate + 2 H+ + N-sulfo-alpha-D-glucosaminyl-[heparan sulfate](n). Also known as: [heparan sulfate]-glucosamine N-sulfotransferase activity, [heparan sulphate]-glucosamine N-sulphotransferase activity, desulfoheparin sulfotransferase activity, heparin-glucosamine N-sulfotransferase activity, heparitin N-sulfotransferase activity, heparitin N-sulphotransferase activity, heparitin sulfotransferase activity, 3'-phosphoadenylyl-sulfate:N-desulfoheparin N-sulfotransferase activity, 3'-phosphoadenylyl-sulfate:[heparan sulfate]-glucosamine N-sulfotransferase activity, 3'-phosphoadenylyl-sulfate:heparitin N-sulfotransferase activity, 3'-phosphoadenylylsulfate:N-desulfoheparin sulfotransferase activity, N-HSST activity, N-desulfoheparin sulfotransferase activity, N-heparan sulfate sulfotransferase activity, PAPS:DSH sulfotransferase activity, PAPS:N-desulfoheparin sulfotransferase activity, glucosaminyl N-deacetylase/N-sulfotransferase activity, heparan sulfate 2-N-sulfotransferase activity, heparan sulfate N-deacetylase/N-sulfotransferase activity, heparin N-deacetylase/N-sulfotransferase activity, heparin N-deacetylase/N-sulphotransferase activity, heparin N-sulfotransferase activity Relationships: is a type of GO:0034483 Sources: EC:2.8.2.8, RHEA:21980 Note: Note that this activity includes EC:2.8.2.12 (deleted from EC).